{
  "term_id": "UNKNOWN:0001",
  "gene_name": "BEN domain-containing protein 4",
  "gene_symbol": "BEND4",
  "term_label": "Unknown molecular function",
  "gene": "UniProtKB:Q6ZU67"
}